mannan biosynthetic process [GO:0046354] (BP) Definition: The chemical reactions and pathways resulting in the formation of mannan, the main hemicellulose of soft (coniferous) wood, made up of D-mannose, D-glucose and D-galactose. Sources: ISBN:0198506732 Also known as: mannan anabolism, mannan biosynthesis, mannan formation, mannan synthesis Relationships: is_a GO:0010412; is a type of GO:0070592 Subtypes: beta-1,2-oligomannoside biosynthetic process [GO:0070136]